{
  "gene": "UniProtKB:P0C7U3",
  "gene_name": "Probable palmitoyltransferase ZDHHC11B",
  "term_label": "Golgi apparatus",
  "gene_symbol": "ZDHHC11B",
  "term_id": "GO:0005794"
}